{
  "gene": "UniProtKB:O75051",
  "gene_name": "Plexin-A2",
  "term_label": "synapse assembly",
  "gene_symbol": "PLXNA2",
  "term_id": "GO:0007416"
}